nucleobase-containing compound biosynthetic process [GO:0034654] (biological process) Also known as: nucleobase, nucleoside, nucleotide and nucleic acid anabolism, nucleobase, nucleoside, nucleotide and nucleic acid biosynthesis, nucleobase, nucleoside, nucleotide and nucleic acid formation, nucleobase, nucleoside, nucleotide and nucleic acid synthesis Sources: GOC:mah Subtypes: GO:0034404, nucleic acid biosynthetic process [GO:0141187], nucleoside phosphate biosynthetic process [GO:1901293] Definition: The chemical reactions and pathways resulting in the formation of nucleobases, nucleosides, nucleotides and nucleic acids. Relationships: is a type of nucleobase-containing compound metabolic process [GO:0006139]; is a type of biosynthetic process [GO:0009058]